response to interleukin-32 [GO:0097395] (biological process) Relationships: is a type of response to cytokine [GO:0034097] Sources: GOC:pr Definition: Any process that results in a change in state or activity of a cell or an organism (in terms of movement, secretion, enzyme production, gene expression, etc.) as a result of an interleukin-32 stimulus. Also known as: response to IL-32 Subtypes: cellular response to interleukin-32 [GO:0097397]